{
  "gene_symbol": "KRT17",
  "term_label": "epithelial cell differentiation",
  "gene_name": "Keratin, type I cytoskeletal 17",
  "term_id": "GO:0030855",
  "gene": "UniProtKB:Q04695"
}